Mullerian duct regression [GO:0001880] (biological process) Relationships: is a type of developmental process involved in reproduction [GO:0003006]; is a type of anatomical structure regression [GO:0060033]; is part of GO:0046661 References: PMID:12368913 Sources: GOC:dph Definition: The process in which the Mullerian ducts, primordia of the oviducts, uterus and upper vagina, undergo regression in male embryos.